{
  "term_id": "UNKNOWN:0002",
  "gene_name": "Coiled-coil domain-containing protein 18",
  "gene_symbol": "CCDC18",
  "gene": "UniProtKB:Q5T9S5",
  "term_label": "Unknown biological process"
}